negative regulation of glomerular filtration by angiotensin [GO:0003106] (biological process) Sources: GOC:dph, GOC:mah, GOC:tb Relationships: is a type of GO:0003083; is part of negative regulation of glomerular filtration [GO:0003105] Definition: The process in which angiotensin directly decreases the rate of glomerular filtration in the kidney. Glomerular filtration is the process whereby blood is filtered by the glomerulus into the renal tubule. Also known as: angiotensin-mediated regulation of glomerular filtration, regulation of glomerular filtration by angiotensin